{
  "gene_name": "Calcineurin subunit B type 2",
  "gene": "UniProtKB:Q96LZ3",
  "term_id": "GO:0097720",
  "term_label": "calcineurin-mediated signaling",
  "gene_symbol": "PPP3R2"
}